inhibition of neuroepithelial cell differentiation [GO:0002085] (BP) Relationships: is a type of regulation of anatomical structure morphogenesis [GO:0022603]; is a type of negative regulation of epithelial cell differentiation [GO:0030857]; is a type of regulation of embryonic development [GO:0045995]; is a type of regulation of timing of cell differentiation [GO:0048505]; negatively regulates neuroepithelial cell differentiation [GO:0060563] Definition: Any process that prevents the activation of neuroepithelial cell differentiation. Neuroepithelial cell differentiation is the process in which epiblast cells acquire specialized features of neuroepithelial cells. Also known as: negative regulation of neural plate formation, repression of premature neural plate formation Subtypes: GO:0061106, negative regulation of odontoblast differentiation [GO:1901330] References: PMID:16678814 Sources: GOC:dph